{
  "gene_symbol": "HUNK",
  "term_label": "protein serine/threonine kinase activity",
  "gene_name": "Hormonally up-regulated neu tumor-associated kinase",
  "gene": "UniProtKB:P57058",
  "term_id": "GO:0004674"
}